interleukin-4 production [GO:0032633] (biological process) Sources: GOC:mah Relationships: is_a GO:0001816 Regulation: regulated by GO:0032673; negatively regulated by negative regulation of interleukin-4 production [GO:0032713]; positively regulated by positive regulation of interleukin-4 production [GO:0032753] Also known as: IL-4 production, interleukin-4 biosynthetic process, interleukin-4 secretion Definition: The appearance of interleukin-4 due to biosynthesis or secretion following a cellular stimulus, resulting in an increase in its intracellular or extracellular levels.